{
  "gene_name": "E3 ubiquitin-protein ligase DTX4",
  "gene": "UniProtKB:Q9Y2E6",
  "term_label": "nucleoplasm",
  "term_id": "GO:0005654",
  "gene_symbol": "DTX4"
}